{
  "term_label": "Unknown molecular function",
  "gene_symbol": "CCDC78",
  "gene_name": "Coiled-coil domain-containing protein 78",
  "term_id": "UNKNOWN:0001",
  "gene": "UniProtKB:A2IDD5"
}